{
  "gene_name": "Androgen receptor",
  "term_id": "GO:0005634",
  "gene": "UniProtKB:P10275",
  "term_label": "nucleus",
  "gene_symbol": "AR"
}